{
  "term_id": "GO:0005615",
  "gene": "UniProtKB:Q9BZM5",
  "gene_symbol": "ULBP2",
  "term_label": "extracellular space",
  "gene_name": "UL16-binding protein 2"
}